ossification [GO:0001503] (biological process) References: PMID:17572649 Sources: GOC:mtg_mpo Also known as: bone biosynthesis, bone formation, osteogenesis Relationships: is a type of multicellular organismal process [GO:0032501] Definition: The formation of bone or of a bony substance, or the conversion of fibrous tissue or of cartilage into bone or a bony substance. Subtypes: direct ossification [GO:0036072], replacement ossification [GO:0036075], ligamentous ossification [GO:0036076], intratendonous ossification [GO:0036077], ossification involved in bone maturation [GO:0043931], GO:0043932 Regulation: regulated by regulation of ossification [GO:0030278]; negatively regulated by GO:0030279; positively regulated by GO:0045778 Note: Note that this term does not have a 'developmental process' parent because ossification isn't necessarily developmental, can also occur as part of bone remodeling. Instead use 'ossification involved in bone maturation ; GO:0043931'.